{
  "term_label": "negative regulation of cytoplasmic translation",
  "term_id": "GO:2000766",
  "gene": "UniProtKB:Q8NE35",
  "gene_symbol": "CPEB3",
  "gene_name": "Cytoplasmic polyadenylation element-binding protein 3"
}